{
  "term_id": "UNKNOWN:0001",
  "gene_name": "Protein Jumonji",
  "gene": "UniProtKB:Q92833",
  "gene_symbol": "JARID2",
  "term_label": "Unknown molecular function"
}